{
  "term_label": "G protein-coupled receptor signaling pathway",
  "gene_name": "Olfactory receptor 5T3",
  "gene_symbol": "OR5T3",
  "term_id": "GO:0007186",
  "gene": "UniProtKB:Q8NGG3"
}